{
  "term_label": "mRNA splicing, via spliceosome",
  "gene": "UniProtKB:Q15695",
  "gene_name": "Putative U2 small nuclear ribonucleoprotein auxiliary factor 35 kDa subunit-related protein 1",
  "gene_symbol": "ZRSR2P1",
  "term_id": "GO:0000398"
}